{
  "term_id": "GO:0070525",
  "gene_symbol": "CTAG2",
  "gene": "UniProtKB:O75638",
  "gene_name": "Cancer_testis antigen 2",
  "term_label": "tRNA threonylcarbamoyladenosine metabolic process"
}